{
  "gene_symbol": "RHOJ",
  "gene_name": "Rho-related GTP-binding protein RhoJ",
  "term_id": "GO:0003924",
  "gene": "UniProtKB:Q9H4E5",
  "term_label": "GTPase activity"
}